{
  "term_id": "GO:0005886",
  "gene_name": "Thrombospondin type-1 domain-containing protein 7B",
  "term_label": "plasma membrane",
  "gene_symbol": "THSD7B",
  "gene": "UniProtKB:Q9C0I4"
}